{
  "gene_name": "Alpha-2B adrenergic receptor",
  "gene_symbol": "ADRA2B",
  "gene": "UniProtKB:P18089",
  "term_label": "epinephrine binding",
  "term_id": "GO:0051379"
}